{
  "gene_name": "Glycogen synthase kinase-3 beta",
  "gene_symbol": "GSK3B",
  "term_id": "GO:0070507",
  "term_label": "regulation of microtubule cytoskeleton organization",
  "gene": "UniProtKB:P49841"
}